{
  "gene": "UniProtKB:P40200",
  "gene_name": "T-cell surface protein tactile",
  "term_label": "Unknown cellular component",
  "term_id": "UNKNOWN:0003",
  "gene_symbol": "CD96"
}